{
  "gene_symbol": "ADGRA3",
  "term_label": "Unknown molecular function",
  "gene": "UniProtKB:Q8IWK6",
  "term_id": "UNKNOWN:0001",
  "gene_name": "Adhesion G protein-coupled receptor A3"
}